{
  "gene_symbol": "EYA1",
  "gene_name": "Eyes absent homolog 1",
  "term_label": "negative regulation of extrinsic apoptotic signaling pathway in absence of ligand",
  "term_id": "GO:2001240",
  "gene": "UniProtKB:Q99502"
}